{
  "gene": "UniProtKB:A0A0J9YWN2",
  "term_id": "UNKNOWN:0002",
  "term_label": "Unknown biological process",
  "gene_name": "Immunoglobulin heavy joining 2 (Fragment)",
  "gene_symbol": "IGHJ2"
}